{
  "gene_symbol": "GNB1L",
  "gene_name": "Guanine nucleotide-binding protein subunit beta-like protein 1",
  "gene": "UniProtKB:Q9BYB4",
  "term_label": "Unknown molecular function",
  "term_id": "UNKNOWN:0001"
}